{
  "term_id": "UNKNOWN:0003",
  "term_label": "Unknown cellular component",
  "gene_symbol": "FUT11",
  "gene_name": "Alpha-(1,3)-fucosyltransferase 11",
  "gene": "UniProtKB:Q495W5"
}